{
  "gene_symbol": "SGIP1",
  "term_id": "UNKNOWN:0001",
  "gene": "UniProtKB:Q9BQI5",
  "term_label": "Unknown molecular function",
  "gene_name": "SH3-containing GRB2-like protein 3-interacting protein 1"
}